peptide antigen transport [GO:0046968] (biological process) References: PMID:15771591 Sources: GOC:add, ISBN:0781735149 Relationships: is a type of peptide transport [GO:0015833]; is part of GO:0048002 Regulation: regulated by regulation of peptide antigen transport [GO:1901039]; negatively regulated by GO:1901040; positively regulated by GO:1901041 Definition: The directed movement of a peptide antigen into, out of or within a cell, or between cells, by means of some agent such as a transporter or pore. The peptide antigen is typically, but not always, processed from an endogenous or exogenous protein.